outer ear morphogenesis [GO:0042473] (biological process) Definition: The process in which the anatomical structures of the outer ear are generated and organized. The outer ear is the part of the ear external to the tympanum (eardrum). It consists of a tube (the external auditory meatus) that directs sound waves on to the tympanum, and may also include the external pinna, which extends beyond the skull. Relationships: is a type of embryonic morphogenesis [GO:0048598]; is part of GO:0042471 Sources: GOC:jl, ISBN:0192801023